actin cortical patch [GO:0030479] (cellular component) Definition: An endocytic patch that consists of an actin-containing structure found at the plasma membrane in cells; formed of networks of branched actin filaments that lie just beneath the plasma membrane and assemble, move, and disassemble rapidly. An example of this is the actin cortical patch found in Saccharomyces cerevisiae. References: PMID:16959963 Sources: GOC:mah, GOC:vw, ISBN:0879693568, ISBN:0879693649 Relationships: is a type of endocytic patch [GO:0061645]; is part of cortical actin cytoskeleton [GO:0030864] Also known as: actin patch